regulation of nucleotide catabolic process [GO:0030811] (biological process) Definition: Any process that modulates the frequency, rate or extent of the chemical reactions and pathways resulting in the breakdown of nucleotides. Sources: GOC:mah Also known as: regulation of nucleotide breakdown, regulation of nucleotide catabolism, regulation of nucleotide degradation Relationships: is a type of regulation of nucleotide metabolic process [GO:0006140]; is a type of regulation of catabolic process [GO:0009894]; regulates nucleotide catabolic process [GO:0009166] Subtypes: regulation of cyclic nucleotide catabolic process [GO:0030805], negative regulation of nucleotide catabolic process [GO:0030812], GO:0030813, regulation of purine nucleotide catabolic process [GO:0033121]